{
  "term_label": "extracellular matrix",
  "gene": "UniProtKB:O60568",
  "gene_name": "Multifunctional procollagen lysine hydroxylase and glycosyltransferase LH3",
  "gene_symbol": "PLOD3",
  "term_id": "GO:0031012"
}